{
  "term_id": "GO:0006890",
  "gene_symbol": "TMEM115",
  "gene_name": "Transmembrane protein 115",
  "term_label": "retrograde vesicle-mediated transport, Golgi to endoplasmic reticulum",
  "gene": "UniProtKB:Q12893"
}